neurotrophin TRK receptor signaling pathway [GO:0048011] (biological process) Definition: The series of molecular signals initiated by neurotrophin binding to its receptor on the surface of a target cell where the receptor possesses tyrosine kinase activity, and ending with the regulation of a downstream cellular process, e.g. transcription. References: PMID:12065629 Sources: GOC:bf, GOC:ceb, GOC:jc, GOC:signaling, Wikipedia:Trk_receptor Also known as: tropomyosin-receptor-kinase signaling, TrkA signaling pathway, TrkB signaling pathway, TrkC signaling pathway Regulation: RO_0002211 by regulation of neurotrophin TRK receptor signaling pathway [GO:0051386]; negatively regulated by negative regulation of neurotrophin TRK receptor signaling pathway [GO:0051387]; positively regulated by positive regulation of neurotrophin TRK receptor signaling pathway [GO:0051388] Relationships: is a type of cell surface receptor protein tyrosine kinase signaling pathway [GO:0007169]; is a type of neurotrophin signaling pathway [GO:0038179]